type 4 serotonin receptor binding [GO:0031829] (molecular function) Also known as: 5-hydroxytryptamine 4 receptor binding, type 4 serotonin receptor ligand Definition: Binding to a type 4 serotonin receptor. Relationships: is a type of G protein-coupled serotonin receptor binding [GO:0031821] Sources: GOC:mah, GOC:nln